{
  "term_id": "GO:0005634",
  "gene": "UniProtKB:Q96FF9",
  "term_label": "nucleus",
  "gene_symbol": "CDCA5",
  "gene_name": "Sororin"
}